{
  "gene_name": "Obscurin",
  "term_id": "GO:0004672",
  "gene": "UniProtKB:Q5VST9",
  "gene_symbol": "OBSCN",
  "term_label": "protein kinase activity"
}